{
  "term_id": "GO:1900118",
  "term_label": "negative regulation of execution phase of apoptosis",
  "gene_name": "Humanin-like 9",
  "gene_symbol": "MTRNR2L9",
  "gene": "UniProtKB:P0CJ76"
}